negative regulation of neuroinflammatory response [GO:0150079] (biological process) Relationships: is_a negative regulation of inflammatory response [GO:0050728]; is a type of GO:0150077; negatively regulates neuroinflammatory response [GO:0150076] References: PMID:11099416, PMID:18164423 Sources: GOC:aruk, GOC:bc Subtypes: negative regulation of astrocyte activation [GO:0061889], negative regulation of microglial cell activation [GO:1903979] Definition: Any process that stops, prevents or reduces the frequency, rate or extent of neuroinflammatory response.